{
  "term_label": "immunoglobulin mediated immune response",
  "term_id": "GO:0016064",
  "gene": "UniProtKB:A0A0J9YVY3",
  "gene_name": "Immunoglobulin heavy variable 7-4-1",
  "gene_symbol": "IGHV7-4-1"
}